maintenance of ciliary planar beating movement pattern [GO:0120221] (biological process) Relationships: is a type of regulation of cilium movement [GO:0003352] References: PMID:26506310 Sources: GOC:krc Definition: Any process involved in maintaining the planar beating pattern of ciliary movement pattern. Connection between the outer doublets and the central pair via the radial spokes constrains ciliary movement to the planar beating pattern. Cilia that lack this connection, such as those in the embryonic node or Kupfer's vesicle, display radial movement. Note: Note that we deem cilium and microtubule-based flagellum to be equivalent.